polar ring of apical complex [GO:0020031] (cellular component) Also known as: anterior polar ring of apical complex, upper polar ring of apical complex Relationships: is a type of cellular anatomical structure [GO:0110165]; is part of apical complex [GO:0020007] Definition: An electron dense ring at the most anterior position of the apical complex, from which the conoid fibers originate; formed during an invasive life cycle stage of an apicomplexan parasite. References: PMID:16518471 Sources: GOC:mb